{
  "term_id": "GO:0004860",
  "gene": "UniProtKB:O60239",
  "gene_symbol": "SH3BP5",
  "term_label": "protein kinase inhibitor activity",
  "gene_name": "SH3 domain-binding protein 5"
}